{
  "term_label": "cytoplasmic microtubule",
  "gene_name": "F-box_WD repeat-containing protein 11",
  "term_id": "GO:0005881",
  "gene_symbol": "FBXW11",
  "gene": "UniProtKB:Q9UKB1"
}